{
  "term_label": "cyclic-di-GMP binding",
  "term_id": "GO:0035438",
  "gene_symbol": "STING1",
  "gene": "UniProtKB:Q86WV6",
  "gene_name": "Stimulator of interferon genes protein"
}